{
  "gene": "UniProtKB:Q86T03",
  "gene_symbol": "PIP4P1",
  "term_id": "GO:0031902",
  "term_label": "late endosome membrane",
  "gene_name": "Type 1 phosphatidylinositol 4,5-bisphosphate 4-phosphatase"
}